{
  "gene_symbol": "HIP1R",
  "term_label": "phosphatidylinositol-3,4-bisphosphate binding",
  "gene": "UniProtKB:O75146",
  "gene_name": "Huntingtin-interacting protein 1-related protein",
  "term_id": "GO:0043325"
}